positive regulation of neural crest cell differentiation [GO:1905294] (biological process) Relationships: is a type of positive regulation of multicellular organismal process [GO:0051240]; is a type of GO:1905292; is a type of positive regulation of stem cell differentiation [GO:2000738]; positively regulates GO:0014033 Definition: Any process that activates or increases the frequency, rate or extent of neural crest cell differentiation. Also known as: up regulation of neural crest cell differentiation, up-regulation of neural crest cell differentiation, upregulation of neural crest cell differentiation, activation of neural crest cell differentiation References: PMID:15073157 Sources: GOC:BHF, GOC:TermGenie, GOC:rl, GO_REF:0000058 Subtypes: positive regulation of neural crest cell fate specification [GO:1905297]